{
  "term_label": "virus receptor activity",
  "gene": "UniProtKB:Q15223",
  "gene_name": "Nectin-1",
  "term_id": "GO:0001618",
  "gene_symbol": "NECTIN1"
}